{
  "gene": "UniProtKB:Q8N4C6",
  "term_id": "GO:0097539",
  "term_label": "ciliary transition fiber",
  "gene_symbol": "NIN",
  "gene_name": "Ninein"
}